{
  "gene_symbol": "ABHD18",
  "gene": "UniProtKB:Q0P651",
  "term_label": "Unknown cellular component",
  "term_id": "UNKNOWN:0003",
  "gene_name": "Protein ABHD18"
}